cellular response to cell wall damage [GO:1990394] (biological process) References: PMID:17287531 Definition: Any process that results in a change in state or activity of a cell (in terms of movement, secretion, enzyme production, gene expression, etc.) as a result of cell wall damage. The process begins with detection of the damage and ends with a change in state or activity of the cell. Relationships: is a type of cellular response to stimulus [GO:0051716]; BFO_0000051 cell wall repair [GO:0071433]